{
  "gene": "UniProtKB:Q8NGC6",
  "gene_name": "Olfactory receptor 4K17",
  "term_label": "Unknown biological process",
  "term_id": "UNKNOWN:0002",
  "gene_symbol": "OR4K17"
}